{
  "gene_symbol": "FOXL1",
  "term_label": "Unknown cellular component",
  "gene": "UniProtKB:Q12952",
  "term_id": "UNKNOWN:0003",
  "gene_name": "Forkhead box protein L1"
}